RNA polymerase I transcription repressor complex [GO:0090570] (cellular component) Definition: A protein complex, located in the nucleus, that possesses activity that prevents or downregulates transcription from a RNA polymerase I promoter. Relationships: is a type of transcription repressor complex [GO:0017053]; is a type of GO:0140513 Sources: GOC:tb